{
  "term_label": "nucleus",
  "term_id": "GO:0005634",
  "gene_name": "Serine_threonine-protein kinase Nek11",
  "gene_symbol": "NEK11",
  "gene": "UniProtKB:Q8NG66"
}